3-phosphoinositide-dependent protein kinase activity [GO:0004676] (molecular function) Note: This reaction requires the presence of a phosphatidylinositol-3-phosphate. Definition: Phosphatidylinositol-3-phosphate-dependent catalysis of the reaction: ATP + a protein = ADP + a phosphoprotein. Sources: GOC:mah Relationships: is a type of protein serine/threonine kinase activity [GO:0004674] Also known as: phosphatidylinositol-3-phosphate protein kinase activity, PDK activity